{
  "term_id": "GO:0007165",
  "gene": "UniProtKB:Q8IYS5",
  "gene_name": "Osteoclast-associated immunoglobulin-like receptor",
  "gene_symbol": "OSCAR",
  "term_label": "signal transduction"
}